{
  "term_id": "GO:0032797",
  "gene": "UniProtKB:Q8WXD5",
  "gene_symbol": "GEMIN6",
  "gene_name": "Gem-associated protein 6",
  "term_label": "SMN complex"
}